{
  "gene": "UniProtKB:C4AMC7",
  "gene_symbol": "WASH3P",
  "term_id": "GO:0055037",
  "gene_name": "Putative WAS protein family homolog 3",
  "term_label": "recycling endosome"
}